{
  "gene_symbol": "ENO1",
  "gene_name": "Alpha-enolase",
  "term_label": "glycolytic process",
  "term_id": "GO:0006096",
  "gene": "UniProtKB:P06733"
}